{
  "term_id": "GO:0071949",
  "gene": "UniProtKB:Q9Y6N5",
  "gene_symbol": "SQOR",
  "gene_name": "Sulfide:quinone oxidoreductase, mitochondrial",
  "term_label": "FAD binding"
}